{
  "gene": "UniProtKB:Q5UE93",
  "gene_name": "Phosphoinositide 3-kinase regulatory subunit 6",
  "term_id": "GO:0005942",
  "term_label": "phosphatidylinositol 3-kinase complex",
  "gene_symbol": "PIK3R6"
}